{
  "term_label": "Unknown molecular function",
  "gene_symbol": "FBXL12",
  "gene": "UniProtKB:Q9NXK8",
  "gene_name": "F-box_LRR-repeat protein 12",
  "term_id": "UNKNOWN:0001"
}